{
  "term_label": "cytoplasm",
  "gene_symbol": "ALDH3B1",
  "gene": "UniProtKB:P43353",
  "gene_name": "Aldehyde dehydrogenase family 3 member B1",
  "term_id": "GO:0005737"
}